{
  "gene": "UniProtKB:P49281",
  "gene_symbol": "SLC11A2",
  "term_label": "plasma membrane",
  "gene_name": "Natural resistance-associated macrophage protein 2",
  "term_id": "GO:0005886"
}